{
  "gene_symbol": "APOBEC2",
  "gene": "UniProtKB:Q9Y235",
  "term_id": "GO:0003723",
  "gene_name": "C-U-editing enzyme APOBEC-2",
  "term_label": "RNA binding"
}